{
  "term_id": "GO:0050767",
  "gene": "UniProtKB:Q5TGS1",
  "term_label": "regulation of neurogenesis",
  "gene_name": "Transcription factor HES-3",
  "gene_symbol": "HES3"
}